{
  "gene_name": "Menin",
  "term_label": "Y-form DNA binding",
  "term_id": "GO:0000403",
  "gene_symbol": "MEN1",
  "gene": "UniProtKB:O00255"
}